{
  "gene_symbol": "DLGAP1",
  "term_id": "GO:0098978",
  "term_label": "glutamatergic synapse",
  "gene": "UniProtKB:O14490",
  "gene_name": "Disks large-associated protein 1"
}